carbonate dehydratase activity [GO:0004089] (MF) Definition: Catalysis of the reaction: hydrogencarbonate + H+ = CO2 + H2O. Sources: EC:4.2.1.1 Also known as: carbonic anhydrase activity, anhydrase activity, carbonate anhydrase activity, carbonate hydro-lyase (carbon-dioxide-forming), carbonate hydro-lyase activity, carbonic acid anhydrase activity, carbonic anhydrase A, carbonic dehydratase activity, carboxyanhydrase activity Relationships: is a type of hydro-lyase activity [GO:0016836]